{
  "term_id": "GO:0050766",
  "gene_symbol": "FCER1G",
  "gene": "UniProtKB:P30273",
  "term_label": "positive regulation of phagocytosis",
  "gene_name": "High affinity immunoglobulin epsilon receptor subunit gamma"
}